{
  "term_id": "GO:0009898",
  "gene_name": "Regulator of G-protein signaling 19",
  "gene": "UniProtKB:P49795",
  "gene_symbol": "RGS19",
  "term_label": "cytoplasmic side of plasma membrane"
}